{
  "gene_name": "Olfactory receptor 5D14",
  "gene_symbol": "OR5D14",
  "term_label": "odorant binding",
  "term_id": "GO:0005549",
  "gene": "UniProtKB:Q8NGL3"
}